{
  "gene": "UniProtKB:Q8N720",
  "term_id": "GO:0006357",
  "gene_symbol": "ZNF655",
  "term_label": "regulation of transcription by RNA polymerase II",
  "gene_name": "Zinc finger protein 655"
}